{
  "term_id": "UNKNOWN:0003",
  "gene_symbol": "UNC79",
  "term_label": "Unknown cellular component",
  "gene": "UniProtKB:Q9P2D8",
  "gene_name": "Protein unc-79 homolog"
}